{
  "gene": "UniProtKB:Q96G21",
  "term_id": "GO:0034457",
  "term_label": "Mpp10 complex",
  "gene_name": "U3 small nucleolar ribonucleoprotein protein IMP4",
  "gene_symbol": "IMP4"
}